{
  "gene_symbol": "AICDA",
  "term_id": "GO:0005634",
  "gene": "UniProtKB:Q9GZX7",
  "gene_name": "Single-stranded DNA cytosine deaminase",
  "term_label": "nucleus"
}